positive regulation of cell proliferation in bone marrow [GO:0071864] (biological process) Definition: A process that activates or increases the frequency, rate or extent of cell proliferation in the bone marrow. References: PMID:17063141 Sources: GOC:mah, GOC:yaf Also known as: positive regulation of bone marrow cell proliferation, up regulation of cell proliferation in bone marrow, up-regulation of cell proliferation in bone marrow, upregulation of cell proliferation in bone marrow, activation of cell proliferation in bone marrow, stimulation of cell proliferation in bone marrow Relationships: is a type of GO:0008284; is a type of regulation of cell proliferation in bone marrow [GO:0071863]; RO_0002213 cell proliferation in bone marrow [GO:0071838]